synaptic vesicle uncoating [GO:0016191] (biological process) Definition: The removal of the protein coat on a synaptic vesicle following the pinching step at the end of budding from the presynaptic membrane. Regulation: regulated by regulation of synaptic vesicle uncoating [GO:1903388]; negatively regulated by negative regulation of synaptic vesicle uncoating [GO:1903389]; positively regulated by GO:1903390 References: PMID:10099709, PMID:24596248 Sources: GOC:curators Also known as: synaptic vesicle coat depolymerization, synaptic vesicle coat protein depolymerization Relationships: is a type of GO:0072318; is part of synaptic vesicle endocytosis [GO:0048488]